branching involved in seminal vesicle morphogenesis [GO:0061683] (biological process) Also known as: gonecyst branching morphogenesis, seminal gland branching morphogenesis, seminal vesicle branching, seminal vesicle branching morphogenesis Definition: The process in which the branching structure of the seminal vesicle is generated and organized. A branch is a division or offshoot from a main stem. Relationships: is a type of morphogenesis of a branching epithelium [GO:0061138]; is part of seminal vesicle epithelium development [GO:0061108]; is part of GO:0061682 References: PMID:16916376 Sources: GOC:dph